{
  "gene_symbol": "STARD10",
  "gene_name": "START domain-containing protein 10",
  "term_id": "GO:0016020",
  "term_label": "membrane",
  "gene": "UniProtKB:Q9Y365"
}